{
  "gene": "UniProtKB:Q96PI1",
  "term_label": "Unknown biological process",
  "gene_symbol": "SPRR4",
  "gene_name": "Small proline-rich protein 4",
  "term_id": "UNKNOWN:0002"
}